{
  "gene_name": "Disintegrin and metalloproteinase domain-containing protein 9",
  "gene": "UniProtKB:Q13443",
  "term_id": "GO:0007179",
  "gene_symbol": "ADAM9",
  "term_label": "transforming growth factor beta receptor signaling pathway"
}